{
  "term_label": "muscle structure development",
  "term_id": "GO:0061061",
  "gene_symbol": "PDLIM2",
  "gene": "UniProtKB:Q96JY6",
  "gene_name": "PDZ and LIM domain protein 2"
}